{
  "term_label": "dynein light intermediate chain binding",
  "gene": "UniProtKB:Q5EBL4",
  "gene_symbol": "RILPL1",
  "gene_name": "RILP-like protein 1",
  "term_id": "GO:0051959"
}